beta-endorphin receptor binding [GO:0071857] (molecular function) Definition: Binding to a beta-endorphin receptor. Sources: GOC:kmv, GOC:mah Relationships: is a type of neuropeptide receptor binding [GO:0071855]